{
  "term_label": "cellular response to lipopolysaccharide",
  "gene_symbol": "IL1F10",
  "gene_name": "Interleukin-1 family member 10",
  "term_id": "GO:0071222",
  "gene": "UniProtKB:Q8WWZ1"
}